{
  "term_id": "GO:0005911",
  "gene_name": "Kin of IRRE-like protein 2",
  "gene_symbol": "KIRREL2",
  "gene": "UniProtKB:Q6UWL6",
  "term_label": "cell-cell junction"
}